{
  "term_label": "Unknown molecular function",
  "gene_name": "F-box only protein 3",
  "gene_symbol": "FBXO3",
  "term_id": "UNKNOWN:0001",
  "gene": "UniProtKB:Q9UK99"
}